positive regulation of saliva secretion [GO:0046878] (biological process) Relationships: is a type of GO:0046877; is a type of positive regulation of secretion [GO:0051047]; is a type of GO:0060456; positively regulates saliva secretion [GO:0046541] Definition: Any process that activates or increases the frequency, rate or extent of the regulated release of saliva. Also known as: up regulation of saliva secretion, up-regulation of saliva secretion, upregulation of saliva secretion, activation of saliva secretion, stimulation of saliva secretion Sources: GOC:ai